{
  "gene": "UniProtKB:P43403",
  "term_label": "protein tyrosine kinase activity",
  "gene_name": "Tyrosine-protein kinase ZAP-70",
  "term_id": "GO:0004713",
  "gene_symbol": "ZAP70"
}